{
  "gene_symbol": "ANKRD44",
  "gene": "UniProtKB:Q8N8A2",
  "term_id": "UNKNOWN:0001",
  "term_label": "Unknown molecular function",
  "gene_name": "Serine_threonine-protein phosphatase 6 regulatory ankyrin repeat subunit B"
}